{
  "term_label": "calcium-dependent phospholipase A2 activity",
  "gene_symbol": "PLA2G4E",
  "term_id": "GO:0047498",
  "gene_name": "Cytosolic phospholipase A2 epsilon",
  "gene": "UniProtKB:Q3MJ16"
}